galactomannan catabolic process [GO:0051682] (biological process) Relationships: is a type of polysaccharide catabolic process [GO:0000272]; is a type of GO:0051069 Sources: GOC:ai Regulation: regulated by regulation of galactomannan catabolic process [GO:2000991]; negatively regulated by negative regulation of galactomannan catabolic process [GO:2000992]; positively regulated by positive regulation of galactomannan catabolic process [GO:2000993] Definition: The chemical reactions and pathways resulting in the breakdown of galactomannan, a polysaccharide composed of D-galactosyl and D-mannosyl. The mannosyl units form the backbone structure (a linear main chain) with the D-galactosyl as single side units.